{
  "gene": "UniProtKB:Q9Y5S2",
  "gene_name": "Serine_threonine-protein kinase MRCK beta",
  "term_id": "GO:0005856",
  "gene_symbol": "CDC42BPB",
  "term_label": "cytoskeleton"
}